{
  "term_label": "Unknown cellular component",
  "term_id": "UNKNOWN:0003",
  "gene_name": "Probable non-functional immunoglobulin heavy variable 3-38-3",
  "gene_symbol": "IGHV3-38-3",
  "gene": "UniProtKB:P0DTE1"
}